{
  "term_id": "UNKNOWN:0001",
  "gene_name": "U3 small nucleolar RNA-associated protein 18 homolog",
  "gene_symbol": "UTP18",
  "gene": "UniProtKB:Q9Y5J1",
  "term_label": "Unknown molecular function"
}